bacteriocin catabolic process [GO:0046225] (biological process) Also known as: bacteriocin breakdown, bacteriocin catabolism, bacteriocin degradation Definition: The chemical reactions and pathways resulting in the breakdown of a bacteriocin, any of a heterogeneous group of polypeptide antibiotics that are secreted by certain bacterial strains and are able to kill cells of other susceptible (frequently related) strains after adsorption at specific receptors on the cell surface. They include the colicins, and their mechanisms of action vary. Relationships: is a type of toxin catabolic process [GO:0009407]; is a type of peptide antibiotic catabolic process [GO:0030652]; is a type of bacteriocin metabolic process [GO:0046224]; is_a detoxification of nitrogen compound [GO:0051410] Sources: GOC:ai